{
  "gene_name": "Leucine-rich repeat transmembrane protein CCDC168",
  "term_id": "UNKNOWN:0001",
  "term_label": "Unknown molecular function",
  "gene": "UniProtKB:Q8NDH2",
  "gene_symbol": "CCDC168"
}